{
  "gene": "UniProtKB:O14772",
  "term_label": "Unknown biological process",
  "gene_name": "Fucose-1-phosphate guanylyltransferase",
  "term_id": "UNKNOWN:0002",
  "gene_symbol": "FPGT"
}